{
  "term_label": "neuron projection morphogenesis",
  "gene_name": "Neuronal tyrosine-phosphorylated phosphoinositide-3-kinase adapter 2",
  "term_id": "GO:0048812",
  "gene_symbol": "NYAP2",
  "gene": "UniProtKB:Q9P242"
}